mannan endo-1,6-alpha-mannosidase activity [GO:0008496] (MF) Definition: Catalysis of the random hydrolysis of (1->6)-alpha-D-mannosidic linkages in unbranched (1->6)-mannans. Sources: EC:3.2.1.101 Also known as: endo-alpha-D-mannosidase activity, 1,6-alpha-D-mannan mannanohydrolase activity, 1,6-beta-D-mannan mannanohydrolase activity, endo-1,6-beta-mannanase activity, endo-alpha-1->6-D-mannanase activity, exo-1,6-beta-mannanase activity, mannan endo-1,6-beta-mannosidase activity Relationships: is a type of alpha-mannosidase activity [GO:0004559]